regulation of germ cell proliferation [GO:1905936] (biological process) Definition: Any process that modulates the frequency, rate or extent of germ cell proliferation. Subtypes: GO:1905937, GO:1905938, regulation of male germ cell proliferation [GO:2000254] References: PMID:15342467 Sources: GOC:TermGenie, GO_REF:0000058 Relationships: is a type of regulation of cell population proliferation [GO:0042127]; is a type of regulation of multicellular organismal process [GO:0051239]; RO_0002211 germ cell proliferation [GO:0036093]